{
  "gene_symbol": "FANCL",
  "gene": "UniProtKB:Q9NW38",
  "term_id": "GO:0005634",
  "term_label": "nucleus",
  "gene_name": "E3 ubiquitin-protein ligase FANCL"
}